{
  "gene": "UniProtKB:P08246",
  "gene_symbol": "ELANE",
  "term_label": "extracellular space",
  "term_id": "GO:0005615",
  "gene_name": "Neutrophil elastase"
}